{
  "gene_symbol": "PACRG",
  "gene": "UniProtKB:Q96M98",
  "gene_name": "Parkin coregulated gene protein",
  "term_id": "GO:0005829",
  "term_label": "cytosol"
}